positive regulation of response to type II interferon [GO:0060332] (biological process) Also known as: positive regulation of response to type II IFN, positive regulation of response to immune interferon, positive regulation of response to interferon-gamma, positive regulation of response to gamma-interferon Subtypes: positive regulation of type II interferon-mediated signaling pathway [GO:0060335] Relationships: is a type of positive regulation of innate immune response [GO:0045089]; is a type of regulation of response to type II interferon [GO:0060330]; is a type of positive regulation of response to cytokine stimulus [GO:0060760]; positively regulates response to type II interferon [GO:0034341] Definition: Any process that increases the rate, frequency or extent of a response to type II interferon (interferon-gamma). Response to interferon gamma is a change in state or activity of a cell or an organism (in terms of movement, secretion, enzyme production, gene expression, etc.) as a result of an interferon-gamma stimulus. Sources: GOC:dph